transport vesicle membrane [GO:0030658] (cellular component) Subtypes: ER to Golgi transport vesicle membrane [GO:0012507], Golgi to ER transport vesicle membrane [GO:0012508], inter-Golgi transport vesicle membrane [GO:0012509], trans-Golgi network transport vesicle membrane [GO:0012510], GO:0060201, clathrin-sculpted glutamate transport vesicle membrane [GO:0060203], GO:0070083, exocytic vesicle membrane [GO:0099501] Also known as: secretory vesicle membrane, constitutive secretory pathway transport vesicle membrane Definition: The lipid bilayer surrounding a transport vesicle. Relationships: is a type of cytoplasmic vesicle membrane [GO:0030659]; is_a bounding membrane of organelle [GO:0098588]; BFO_0000050 transport vesicle [GO:0030133] Sources: GOC:mah